{
  "gene_symbol": "UBE2L3",
  "term_label": "ubiquitin-dependent protein catabolic process",
  "gene": "UniProtKB:P68036",
  "gene_name": "Ubiquitin-conjugating enzyme E2 L3",
  "term_id": "GO:0006511"
}